{
  "gene_symbol": "FAM90A16",
  "gene_name": "Protein FAM90A16",
  "term_label": "Unknown molecular function",
  "term_id": "UNKNOWN:0001",
  "gene": "UniProtKB:P0DV73"
}